{
  "gene_symbol": "ZNF875",
  "gene_name": "Zinc finger protein 875",
  "term_label": "regulation of transcription by RNA polymerase II",
  "term_id": "GO:0006357",
  "gene": "UniProtKB:P10072"
}